localization of cell [GO:0051674] (biological process) Definition: Any process in which a cell is transported to, and/or maintained in, a specific location. Also known as: cell localization, establishment and maintenance of cell localization, establishment and maintenance of localization of cell, localisation of cell Relationships: is a type of cellular process [GO:0009987]; is a type of localization [GO:0051179] Sources: GOC:ai Subtypes: oocyte localization involved in germarium-derived egg chamber formation [GO:0030720], GO:0035852